{
  "gene": "UniProtKB:Q9UKB1",
  "gene_symbol": "FBXW11",
  "gene_name": "F-box_WD repeat-containing protein 11",
  "term_label": "neuronal cell body",
  "term_id": "GO:0043025"
}